{
  "term_id": "GO:0045202",
  "gene_name": "CHRNA7-FAM7A fusion protein",
  "gene_symbol": "CHRFAM7A",
  "gene": "UniProtKB:Q494W8",
  "term_label": "synapse"
}